negative regulation of cell-matrix adhesion [GO:0001953] (biological process) Also known as: down regulation of cell-matrix adhesion, down-regulation of cell-matrix adhesion, downregulation of cell-matrix adhesion, inhibition of cell-matrix adhesion Relationships: is a type of regulation of cell-matrix adhesion [GO:0001952]; is a type of GO:0010812; negatively regulates cell-matrix adhesion [GO:0007160] Definition: Any process that stops, prevents, or reduces the rate or extent of cell adhesion to the extracellular matrix. Sources: GOC:hjd Subtypes: negative regulation of focal adhesion assembly [GO:0051895], negative regulation of endothelial cell-matrix adhesion [GO:1904905], negative regulation of smooth muscle cell-matrix adhesion [GO:2000098]